{
  "term_id": "GO:0097602",
  "gene_name": "DCN1-like protein 3",
  "gene_symbol": "DCUN1D3",
  "term_label": "cullin family protein binding",
  "gene": "UniProtKB:Q8IWE4"
}